{
  "gene": "UniProtKB:A8MTQ0",
  "gene_name": "Homeobox protein notochord",
  "term_id": "GO:0007417",
  "gene_symbol": "NOTO",
  "term_label": "central nervous system development"
}